{
  "gene_symbol": "MYO1D",
  "gene_name": "Unconventional myosin-Id",
  "gene": "UniProtKB:O94832",
  "term_id": "GO:0005886",
  "term_label": "plasma membrane"
}